{
  "term_label": "transmembrane signaling receptor activity",
  "gene_name": "Fas apoptotic inhibitory molecule 3",
  "gene": "UniProtKB:O60667",
  "term_id": "GO:0004888",
  "gene_symbol": "FCMR"
}